{
  "gene_symbol": "SETBP1",
  "gene": "UniProtKB:Q9Y6X0",
  "term_label": "nucleoplasm",
  "gene_name": "SET-binding protein",
  "term_id": "GO:0005654"
}